regulation of retinoic acid biosynthetic process [GO:1900052] (BP) Relationships: is a type of regulation of ketone metabolic process [GO:0010565]; is a type of regulation of isoprenoid metabolic process [GO:0019747]; is_a regulation of vitamin metabolic process [GO:0030656]; is_a regulation of hormone metabolic process [GO:0032350]; is a type of GO:0046890; regulates GO:0002138 Subtypes: GO:1900053, positive regulation of retinoic acid biosynthetic process [GO:1900054] Also known as: regulation of retinoic acid anabolic process Sources: GOC:TermGenie, GOC:yaf Definition: Any process that modulates the frequency, rate or extent of retinoic acid biosynthetic process.